{
  "gene": "UniProtKB:P54619",
  "gene_symbol": "PRKAG1",
  "gene_name": "5'-AMP-activated protein kinase subunit gamma-1",
  "term_id": "GO:0019887",
  "term_label": "protein kinase regulator activity"
}